{
  "term_label": "regulation of transcription by RNA polymerase II",
  "term_id": "GO:0006357",
  "gene": "UniProtKB:Q8WYK2",
  "gene_symbol": "JDP2",
  "gene_name": "Jun dimerization protein 2"
}